{
  "term_label": "Unknown cellular component",
  "term_id": "UNKNOWN:0003",
  "gene_name": "Inter-alpha-trypsin inhibitor heavy chain H4",
  "gene_symbol": "ITIH4",
  "gene": "UniProtKB:Q14624"
}